{
  "gene_symbol": "CREM",
  "gene_name": "cAMP-responsive element modulator",
  "term_id": "GO:0006357",
  "term_label": "regulation of transcription by RNA polymerase II",
  "gene": "UniProtKB:Q03060"
}